pteridine oxidase activity [GO:0050227] (molecular function) Sources: RHEA:12777 Also known as: 2-amino-4-hydroxypteridine:oxygen oxidoreductase (7-hydroxylating) Definition: Catalysis of the reaction: 2-amino-4-hydroxypteridine + O2 = 2-amino-4,7-dihydroxypteridine + unknown. Relationships: is a type of oxidoreductase activity, acting on CH or CH2 groups, oxygen as acceptor [GO:0016727]